{
  "term_id": "UNKNOWN:0003",
  "gene_name": "Small integral membrane protein 47",
  "gene": "UniProtKB:D0EPY3",
  "gene_symbol": "SMIM47",
  "term_label": "Unknown cellular component"
}